tRNA 2'-phosphotransferase activity [GO:0000215] (molecular function) Relationships: is a type of GO:0016773; is a type of GO:0140101 Definition: Catalysis of the reaction: 2'-phospho-[ligated tRNA] + NAD+ = mature tRNA + ADP ribose 1'',2''-phosphate + nicotinamide + H2O. This reaction is the transfer of the splice junction 2-phosphate from ligated tRNA to NAD+ to produce ADP-ribose 1'-2' cyclic phosphate. References: PMID:9148937 Sources: EC:2.7.1.160 Also known as: 2'-phosphotransferase activity, yeast 2'-phosphotransferase activity, 2'-phospho-[ligated tRNA]:NAD+ phosphotransferase activity, 2'-phospho-tRNA:NAD+ phosphotransferase activity, Tpt1, Tpt1p